{
  "term_id": "GO:0032797",
  "gene": "UniProtKB:O14893",
  "term_label": "SMN complex",
  "gene_symbol": "GEMIN2",
  "gene_name": "Gem-associated protein 2"
}